{
  "gene_name": "Probable non-functional immunoglobulin heavy variable 3-16",
  "gene": "UniProtKB:A0A0C4DH30",
  "term_label": "antigen binding",
  "gene_symbol": "IGHV3-16",
  "term_id": "GO:0003823"
}